retrograde axonal protein transport [GO:0099642] (biological process) Definition: The directed movement of proteins along microtubules from the cell periphery toward the cell body in nerve cell axons. Sources: ISBN:0815316194 Also known as: retrograde axon cargo transport Relationships: is a type of retrograde axonal transport [GO:0008090]; is_a axo-dendritic protein transport [GO:0099640]